{
  "gene_symbol": "SYT15",
  "gene_name": "Synaptotagmin-15",
  "term_label": "SNARE binding",
  "gene": "UniProtKB:Q9BQS2",
  "term_id": "GO:0000149"
}